negative regulation of blood coagulation, extrinsic pathway [GO:2000264] (biological process) Relationships: is a type of negative regulation of blood coagulation [GO:0030195]; is a type of GO:2000258; is a type of GO:2000263; negatively regulates blood coagulation, extrinsic pathway [GO:0007598] Definition: Any process that stops, prevents or reduces the frequency, rate or extent of blood coagulation, extrinsic pathway. Sources: GOC:mah